inflorescence development [GO:0010229] (biological process) Definition: The process whose specific outcome is the progression of an inflorescence over time, from its formation to the mature structure. Sources: GOC:tb Relationships: is a type of reproductive shoot system development [GO:0090567]